{
  "gene_name": "Nuclear ubiquitous casein and cyclin-dependent kinase substrate 1",
  "term_id": "GO:0003690",
  "term_label": "double-stranded DNA binding",
  "gene_symbol": "NUCKS1",
  "gene": "UniProtKB:Q9H1E3"
}